maturation of 5.8S rRNA [GO:0000460] (biological process) Relationships: is_a rRNA processing [GO:0006364] Definition: Any process involved in the maturation of a precursor 5.8S ribosomal RNA (rRNA) molecule into a mature 5.8S rRNA molecule. Subtypes: GO:0000466, maturation of 5.8S rRNA from tetracistronic rRNA transcript (SSU-rRNA, 5.8S rRNA, 2S rRNA, LSU-rRNA) [GO:0000487] Sources: GOC:curators